regulation of interleukin-18-mediated signaling pathway [GO:2000492] (biological process) Also known as: regulation of interleukin-18-mediated signalling pathway Subtypes: GO:2000493, GO:2000494 Sources: GOC:obol Definition: Any process that modulates the frequency, rate or extent of interleukin-18-mediated signaling pathway. Relationships: is_a regulation of cytokine-mediated signaling pathway [GO:0001959]; regulates interleukin-18-mediated signaling pathway [GO:0035655]